{
  "gene_name": "Large ribosomal subunit protein bL35m",
  "gene": "UniProtKB:Q9NZE8",
  "term_label": "Unknown biological process",
  "gene_symbol": "MRPL35",
  "term_id": "UNKNOWN:0002"
}